{
  "gene_symbol": "MAP1B",
  "gene_name": "Microtubule-associated protein 1B",
  "gene": "UniProtKB:P46821",
  "term_id": "GO:0043025",
  "term_label": "neuronal cell body"
}